{
  "term_id": "GO:0008270",
  "gene": "UniProtKB:P04196",
  "term_label": "zinc ion binding",
  "gene_symbol": "HRG",
  "gene_name": "Histidine-rich glycoprotein"
}